positive regulation of aldosterone biosynthetic process [GO:0032349] (biological process) Also known as: up regulation of aldosterone biosynthetic process, up-regulation of aldosterone biosynthetic process, upregulation of aldosterone biosynthetic process, activation of aldosterone biosynthetic process, stimulation of aldosterone biosynthetic process Definition: Any process that activates or increases the frequency, rate or extent of the chemical reactions and pathways resulting in the formation of aldosterone. Sources: GOC:mah Relationships: is_a GO:0032347; is a type of GO:0090031; is a type of positive regulation of alcohol biosynthetic process [GO:1902932]; positively regulates aldosterone biosynthetic process [GO:0032342]